{
  "gene_name": "UDP-N-acetylglucosamine--peptide N-acetylglucosaminyltransferase 110 kDa subunit",
  "term_label": "protein O-linked glycosylation",
  "gene_symbol": "OGT",
  "term_id": "GO:0006493",
  "gene": "UniProtKB:O15294"
}